xanthosine catabolic process [GO:1903228] (biological process) Relationships: is a type of purine ribonucleoside catabolic process [GO:0046130] References: PMID:7007809, PMID:7559336 Sources: GOC:TermGenie, GO_REF:0000068 Definition: The chemical reactions and pathways resulting in the breakdown of xanthosine. Also known as: xanthosine breakdown, xanthosine catabolism, xanthosine degradation